{
  "gene": "UniProtKB:Q9NZP8",
  "gene_symbol": "C1RL",
  "term_id": "GO:0005615",
  "gene_name": "Complement C1r subcomponent-like protein",
  "term_label": "extracellular space"
}